{
  "gene_name": "Destrin",
  "term_id": "GO:0005737",
  "gene": "UniProtKB:P60981",
  "term_label": "cytoplasm",
  "gene_symbol": "DSTN"
}